{
  "gene": "UniProtKB:Q9UGM3",
  "term_label": "extracellular space",
  "gene_name": "Deleted in malignant brain tumors 1 protein",
  "gene_symbol": "DMBT1",
  "term_id": "GO:0005615"
}